{
  "gene_name": "Nuclear distribution protein nudE-like 1",
  "gene": "UniProtKB:Q9GZM8",
  "term_label": "establishment of mitotic spindle orientation",
  "gene_symbol": "NDEL1",
  "term_id": "GO:0000132"
}